{
  "gene_symbol": "ZNF319",
  "gene_name": "Zinc finger protein 319",
  "term_id": "GO:0006357",
  "gene": "UniProtKB:Q9P2F9",
  "term_label": "regulation of transcription by RNA polymerase II"
}